{
  "term_label": "Unknown cellular component",
  "gene_symbol": "ST8SIA2",
  "gene": "UniProtKB:Q92186",
  "gene_name": "Alpha-2,8-sialyltransferase 8B",
  "term_id": "UNKNOWN:0003"
}